alphaV-beta6 integrin-TGFbeta-3 complex [GO:0071099] (cellular component) Relationships: is a type of GO:0098797 References: PMID:11821050 Also known as: ITGAV-ITGB6-TFGB3 complex Definition: A protein complex that consists of an alphaV-beta6 integrin complex bound to transforming growth factor beta-3 (TGFbeta-3).